{
  "gene_name": "rRNA methyltransferase 3, mitochondrial",
  "term_id": "UNKNOWN:0003",
  "gene": "UniProtKB:Q9HC36",
  "term_label": "Unknown cellular component",
  "gene_symbol": "MRM3"
}